{
  "gene_name": "Annexin A4",
  "gene_symbol": "ANXA4",
  "term_label": "cytoplasm",
  "term_id": "GO:0005737",
  "gene": "UniProtKB:P09525"
}